{
  "gene_name": "DENN domain-containing protein 4C",
  "gene": "UniProtKB:Q5VZ89",
  "term_id": "GO:0032483",
  "gene_symbol": "DENND4C",
  "term_label": "regulation of Rab protein signal transduction"
}